{
  "gene_symbol": "TAF5L",
  "term_id": "GO:0000124",
  "gene_name": "TAF5-like RNA polymerase II p300_CBP-associated factor-associated factor 65 kDa subunit 5L",
  "gene": "UniProtKB:O75529",
  "term_label": "SAGA complex"
}